brevianamide F biosynthetic process [GO:1900805] (biological process) Definition: The chemical reactions and pathways resulting in the formation of brevianamide F. Brevianamide F is the biosynthetic precursor of a large family of biologically active prenylated tryptophan-proline 2,5-diketopiperazines that are produced by some fungi. References: PMID:16755625, PMID:17464044 Sources: GOC:TermGenie, GOC:di Also known as: brevianamide F anabolism, brevianamide F biosynthesis, brevianamide F formation, brevianamide F synthesis, brevianamide F metabolic process, C16H17N3O2 anabolism, C16H17N3O2 biosynthesis, C16H17N3O2 biosynthetic process, C16H17N3O2 formation, C16H17N3O2 synthesis, L-prolyl-L-tryptophan anhydride anabolism, L-prolyl-L-tryptophan anhydride biosynthesis, L-prolyl-L-tryptophan anhydride biosynthetic process, L-prolyl-L-tryptophan anhydride formation, L-prolyl-L-tryptophan anhydride synthesis, L-tryptophyl-L-proline cyclic anhydride anabolism, L-tryptophyl-L-proline cyclic anhydride biosynthesis, L-tryptophyl-L-proline cyclic anhydride biosynthetic process, L-tryptophyl-L-proline cyclic anhydride formation, L-tryptophyl-L-proline cyclic anhydride synthesis, cyclo-(Trp-Pro) anabolism, cyclo-(Trp-Pro) biosynthesis, cyclo-(Trp-Pro) biosynthetic process, cyclo-(Trp-Pro) formation, cyclo-(Trp-Pro) synthesis, cyclo-L-Trp-L-Pro anabolism, cyclo-L-Trp-L-Pro biosynthesis, cyclo-L-Trp-L-Pro biosynthetic process, cyclo-L-Trp-L-Pro formation, cyclo-L-Trp-L-Pro synthesis, cyclo-L-tryptophanyl-L-proline anabolism, cyclo-L-tryptophanyl-L-proline biosynthesis, cyclo-L-tryptophanyl-L-proline biosynthetic process, cyclo-L-tryptophanyl-L-proline formation, cyclo-L-tryptophanyl-L-proline synthesis, tryptophan-proline diketopiperazine anabolism, tryptophan-proline diketopiperazine biosynthesis, tryptophan-proline diketopiperazine biosynthetic process, tryptophan-proline diketopiperazine formation, tryptophan-proline diketopiperazine synthesis Relationships: is a type of GO:0035835; is a type of indole-containing compound biosynthetic process [GO:0042435]; is_a GO:0043604